{
  "term_label": "Unknown cellular component",
  "gene": "UniProtKB:Q99674",
  "gene_name": "Cell growth regulator with EF hand domain protein 1",
  "gene_symbol": "CGREF1",
  "term_id": "UNKNOWN:0003"
}